{
  "term_label": "Unknown molecular function",
  "gene_name": "Small integral membrane protein 26",
  "gene_symbol": "SMIM26",
  "term_id": "UNKNOWN:0001",
  "gene": "UniProtKB:A0A096LP01"
}